{
  "term_label": "Unknown molecular function",
  "gene_symbol": "LY86",
  "gene_name": "Lymphocyte antigen 86",
  "term_id": "UNKNOWN:0001",
  "gene": "UniProtKB:O95711"
}